{
  "gene_symbol": "FAU",
  "term_label": "structural constituent of ribosome",
  "gene_name": "Ubiquitin-like FUBI-ribosomal protein eS30 fusion protein",
  "gene": "UniProtKB:P62861",
  "term_id": "GO:0003735"
}